{
  "gene": "UniProtKB:Q96P20",
  "term_id": "GO:0043565",
  "term_label": "sequence-specific DNA binding",
  "gene_symbol": "NLRP3",
  "gene_name": "NACHT, LRR and PYD domains-containing protein 3"
}